{
  "term_id": "GO:0005794",
  "gene": "UniProtKB:P51159",
  "gene_name": "Ras-related protein Rab-27A",
  "gene_symbol": "RAB27A",
  "term_label": "Golgi apparatus"
}